{
  "term_id": "UNKNOWN:0003",
  "gene": "UniProtKB:Q6UWF5",
  "gene_name": "Putative uncharacterized protein UNQ5815_PRO19632",
  "gene_symbol": "UNQ5815_PRO19632",
  "term_label": "Unknown cellular component"
}